{
  "gene": "UniProtKB:Q6P3S6",
  "term_label": "SCF ubiquitin ligase complex",
  "gene_symbol": "FBXO42",
  "term_id": "GO:0019005",
  "gene_name": "F-box only protein 42"
}